{
  "term_id": "GO:0045324",
  "gene": "UniProtKB:Q9UQN3",
  "term_label": "late endosome to vacuole transport",
  "gene_symbol": "CHMP2B",
  "gene_name": "Charged multivesicular body protein 2b"
}